heterochromatin organization [GO:0070828] (biological process) Also known as: heterochromatin organisation Sources: GOC:mah Definition: Any process that results in the specification, formation or maintenance of the physical structure of eukaryotic heterochromatin, a compact and highly condensed form of chromatin. Subtypes: heterochromatin boundary formation [GO:0033696] Regulation: RO_0002211 by regulation of heterochromatin organization [GO:0120261]; negatively regulated by negative regulation of heterochromatin organization [GO:0120262]; positively regulated by positive regulation of heterochromatin organization [GO:0120263] Relationships: is a type of chromatin organization [GO:0006325]